regulated exocytosis [GO:0045055] (biological process) Definition: A process of exocytosis in which soluble proteins and other substances are initially stored in secretory vesicles for later release. It is found mainly in cells that are specialized for secreting products such as hormones, neurotransmitters, or digestive enzymes rapidly on demand. Sources: GOC:mah, ISBN:0716731363 Also known as: regulated secretory pathway Relationships: is a type of GO:0006887 Subtypes: platelet degranulation [GO:0002576], synaptic vesicle exocytosis [GO:0016079], calcium-ion regulated exocytosis [GO:0017156], leukocyte degranulation [GO:0043299], GO:0070177 Regulation: regulated by GO:1903305; negatively regulated by negative regulation of regulated secretory pathway [GO:1903306]; positively regulated by positive regulation of regulated secretory pathway [GO:1903307]